{
  "gene_symbol": "ETF1",
  "gene_name": "Eukaryotic peptide chain release factor subunit 1",
  "term_id": "GO:0002184",
  "gene": "UniProtKB:P62495",
  "term_label": "cytoplasmic translational termination"
}